{
  "gene_name": "Ubiquitin carboxyl-terminal hydrolase 26",
  "gene_symbol": "USP26",
  "term_label": "G1/S transition of mitotic cell cycle",
  "gene": "UniProtKB:Q9BXU7",
  "term_id": "GO:0000082"
}